{
  "gene_symbol": "HSPBP1",
  "term_id": "UNKNOWN:0002",
  "gene": "UniProtKB:Q9NZL4",
  "term_label": "Unknown biological process",
  "gene_name": "Hsp70-binding protein 1"
}